{
  "term_id": "UNKNOWN:0002",
  "gene_symbol": "OR4A8",
  "term_label": "Unknown biological process",
  "gene_name": "Olfactory receptor 4A8",
  "gene": "UniProtKB:P0C604"
}